{
  "gene": "UniProtKB:Q9HB75",
  "gene_name": "p53-induced death domain-containing protein 1",
  "term_label": "Unknown molecular function",
  "term_id": "UNKNOWN:0001",
  "gene_symbol": "PIDD1"
}